clustering of voltage-gated potassium channels [GO:0045163] (biological process) Definition: The process in which voltage-gated potassium channels become localized together in high densities. In animals, voltage-gated potassium (Kv) channels are clustered beneath the myelin sheath in regions immediately adjacent to paranodes, called juxtaparanodes, and along the inner mesaxon within the internode. References: PMID:11456440 Also known as: Kv channel clustering, clustering of voltage gated potassium channels, clustering of voltage-dependent potassium channels, voltage-gated potassium channel clustering Relationships: is a type of GO:0045161